{
  "term_label": "olfactory receptor activity",
  "gene": "UniProtKB:Q8NGC0",
  "term_id": "GO:0004984",
  "gene_symbol": "OR5AU1",
  "gene_name": "Olfactory receptor 5AU1"
}